{
  "gene": "UniProtKB:Q8N7Q3",
  "gene_symbol": "ZNF676",
  "term_label": "RNA polymerase II cis-regulatory region sequence-specific DNA binding",
  "term_id": "GO:0000978",
  "gene_name": "Zinc finger protein 676"
}